{
  "term_id": "GO:0006357",
  "gene": "UniProtKB:P98168",
  "term_label": "regulation of transcription by RNA polymerase II",
  "gene_name": "Zinc finger X-linked protein ZXDA",
  "gene_symbol": "ZXDA"
}